L-leucine N-acetyltransferase activity [GO:0050050] (molecular function) Also known as: acetyl-CoA:L-leucine N-acetyltransferase activity, leucine acetyltransferase activity Definition: Catalysis of the reaction: L-leucine + acetyl-CoA = N-acetyl-L-leucine + CoA + H+. Relationships: is a type of L-amino-acid N-acetyltransferase activity [GO:0140085] Sources: EC:2.3.1.66, RHEA:20089